interleukin-1 alpha production [GO:0032610] (biological process) Also known as: IL-1 alpha production, interleukin-1 alpha biosynthetic process, interleukin-1 alpha secretion Definition: The appearance of interleukin-1 alpha due to biosynthesis or secretion following a cellular stimulus, resulting in an increase in its intracellular or extracellular levels. Regulation: regulated by regulation of interleukin-1 alpha production [GO:0032650]; negatively regulated by negative regulation of interleukin-1 alpha production [GO:0032690]; positively regulated by GO:0032730 Relationships: is a type of GO:0032612 Sources: GOC:mah